{
  "gene_name": "5-hydroxytryptamine receptor 1D",
  "gene": "UniProtKB:P28221",
  "term_label": "chemical synaptic transmission",
  "term_id": "GO:0007268",
  "gene_symbol": "HTR1D"
}